{
  "gene_symbol": "CTC1",
  "gene_name": "CST complex subunit CTC1",
  "term_label": "telomere maintenance via telomere lengthening",
  "term_id": "GO:0010833",
  "gene": "UniProtKB:Q2NKJ3"
}